CSF1-CSF1R complex [GO:1990682] (cellular component) References: PMID:19017797 Sources: GOC:BHF, GOC:bf, GOC:nc Definition: A protein complex consisting of a macrophage colony-stimulating factor (CSF1, also called M-CSF) dimer bound to a dimerized receptor (CSF1R, also called FMS). Receptor dimerization requires the presence of the ligand. Relationships: is a type of protein-containing complex [GO:0032991] Also known as: CSF1:C-FMS complex, M-CSF:FMS complex, macrophage colony-stimulating factor:receptor complex, M-CSF:C-FMS complex, M-CSF:CSF1R complex